positive regulation of epithelial to mesenchymal transition [GO:0010718] (biological process) Subtypes: GO:0060808, positive regulation of cardiac epithelial to mesenchymal transition [GO:0062043], positive regulation of neural crest formation [GO:0090300] Relationships: is a type of GO:0010717; is_a positive regulation of cell differentiation [GO:0045597]; is a type of GO:0051240; positively regulates epithelial to mesenchymal transition [GO:0001837] Sources: GOC:BHF, GOC:dph, GOC:tb Definition: Any process that increases the rate, frequency, or extent of epithelial to mesenchymal transition. Epithelial to mesenchymal transition is where an epithelial cell loses apical/basolateral polarity, severs intercellular adhesive junctions, degrades basement membrane components and becomes a migratory mesenchymal cell.